{
  "gene_symbol": "BIN3",
  "gene": "UniProtKB:Q9NQY0",
  "term_id": "GO:0015629",
  "gene_name": "Bridging integrator 3",
  "term_label": "actin cytoskeleton"
}